{
  "gene": "UniProtKB:Q5RI15",
  "gene_symbol": "COX20",
  "term_label": "mitochondrion",
  "gene_name": "Cytochrome c oxidase assembly protein COX20, mitochondrial",
  "term_id": "GO:0005739"
}